D-malate dehydrogenase (decarboxylating) (NAD+) activity [GO:0046553] (MF) Definition: Catalysis of the reaction: (R)-malate + NAD+ = CO2 + NADH + pyruvate. Also known as: (R)-malate:NAD+ oxidoreductase (decarboxylating), D-malate dehydrogenase activity, D-malic enzyme, bifunctional L(+)-tartrate dehydrogenase-D(+)-malate (decarboxylating) Relationships: is a type of malate dehydrogenase activity [GO:0016615]; is a type of oxidoreductase activity, acting on the CH-OH group of donors, NAD or NADP as acceptor [GO:0016616] Sources: RHEA:18365